{
  "gene": "UniProtKB:Q8WXI2",
  "term_id": "GO:0099084",
  "gene_name": "Connector enhancer of kinase suppressor of ras 2",
  "term_label": "postsynaptic specialization organization",
  "gene_symbol": "CNKSR2"
}